positive regulation of chemokine (C-C motif) ligand 6 production [GO:0035533] (biological process) Definition: Any process that activates or increases the frequency, rate, or extent of production of chemokine (C-C motif) ligand 6 (CCL6). Sources: GOC:add, GOC:bf Also known as: positive regulation of CCL6 production, positive regulation of chemokine (C-C motif) ligand 6 secretion Relationships: is a type of positive regulation of chemokine production [GO:0032722]; is_a regulation of chemokine (C-C motif) ligand 6 production [GO:0035531]; positively regulates chemokine (C-C motif) ligand 6 production [GO:0035530]